negative regulation of post-transcriptional gene silencing by regulatory ncRNA [GO:1900369] (biological process) Definition: Any process that stops, prevents or reduces the frequency, rate or extent of post-transcriptional gene silencing by RNA. Relationships: is a type of negative regulation of post-transcriptional gene silencing [GO:0060149]; is a type of negative regulation of gene silencing by regulatory ncRNA [GO:0060967]; is_a regulation of post-transcriptional gene silencing by regulatory ncRNA [GO:1900368]; negatively regulates regulatory ncRNA-mediated post-transcriptional gene silencing [GO:0035194] Subtypes: negative regulation of miRNA-mediated gene silencing [GO:0060965] Also known as: down regulation of RNA interference, down regulation of RNAi, down-regulation of RNA interference, down-regulation of RNAi, downregulation of RNA interference, downregulation of RNAi, inhibition of RNAi, negative regulation of PTGS, negative regulation of RNA interference, negative regulation of RNAi, inhibition of RNA interference, negative regulation of posttranscriptional gene silencing by siRNA, negative regulation of post-transcriptional gene silencing by RNA, negative regulation of post-transcriptional gene silencing by ncRNA References: PMID:22412382 Sources: GOC:TermGenie, GOC:kmv